{
  "term_id": "GO:0016324",
  "term_label": "apical plasma membrane",
  "gene_symbol": "UPK2",
  "gene": "UniProtKB:O00526",
  "gene_name": "Uroplakin-2"
}